{
  "gene_name": "Major centromere autoantigen B",
  "term_id": "UNKNOWN:0002",
  "term_label": "Unknown biological process",
  "gene_symbol": "CENPB",
  "gene": "UniProtKB:P07199"
}